{
  "gene_symbol": "PLEKHA8P1",
  "term_id": "GO:1902387",
  "gene": "UniProtKB:O95397",
  "gene_name": "Putative protein PLEKHA9",
  "term_label": "ceramide 1-phosphate binding"
}